nuclear membrane reassembly [GO:0031468] (biological process) Subtypes: mitotic nuclear membrane reassembly [GO:0007084], GO:0051333 Sources: GOC:mah Also known as: nuclear envelope reassembly Relationships: is_a membrane assembly [GO:0071709]; is a type of GO:0071763 Definition: The reformation of the nuclear membranes following their breakdown in the context of a normal process.